{
  "gene": "UniProtKB:Q8NEM8",
  "gene_name": "Cytosolic carboxypeptidase 3",
  "term_id": "GO:0004181",
  "gene_symbol": "AGBL3",
  "term_label": "metallocarboxypeptidase activity"
}